{
  "gene_symbol": "ARHGAP24",
  "term_id": "GO:1900028",
  "gene": "UniProtKB:Q8N264",
  "gene_name": "Rho GTPase-activating protein 24",
  "term_label": "negative regulation of ruffle assembly"
}